{
  "term_label": "Unknown biological process",
  "gene_symbol": "PRAF2",
  "gene": "UniProtKB:O60831",
  "term_id": "UNKNOWN:0002",
  "gene_name": "PRA1 family protein 2"
}